{
  "term_label": "extracellular space",
  "term_id": "GO:0005615",
  "gene": "UniProtKB:P43121",
  "gene_symbol": "MCAM",
  "gene_name": "Cell surface glycoprotein MUC18"
}